{
  "term_id": "GO:0008104",
  "gene_name": "Partitioning defective 3 homolog B",
  "gene": "UniProtKB:Q8TEW8",
  "gene_symbol": "PARD3B",
  "term_label": "intracellular protein localization"
}